{
  "term_label": "extracellular matrix organization",
  "term_id": "GO:0030198",
  "gene": "UniProtKB:Q15582",
  "gene_name": "Transforming growth factor-beta-induced protein ig-h3",
  "gene_symbol": "TGFBI"
}